{
  "term_id": "UNKNOWN:0002",
  "term_label": "Unknown biological process",
  "gene_name": "Immunoglobulin superfamily member 8",
  "gene_symbol": "IGSF8",
  "gene": "UniProtKB:Q969P0"
}